{
  "gene": "UniProtKB:Q9C056",
  "gene_symbol": "NKX6-2",
  "gene_name": "Homeobox protein Nkx-6.2",
  "term_id": "GO:0005634",
  "term_label": "nucleus"
}